{
  "gene_name": "Tubulin alpha-1B chain",
  "gene_symbol": "TUBA1B",
  "gene": "UniProtKB:P68363",
  "term_id": "GO:0005525",
  "term_label": "GTP binding"
}